{
  "gene": "UniProtKB:O75600",
  "gene_symbol": "GCAT",
  "term_id": "UNKNOWN:0001",
  "gene_name": "2-amino-3-ketobutyrate coenzyme A ligase, mitochondrial",
  "term_label": "Unknown molecular function"
}